protein localization to peroxisome [GO:0072662] (BP) Relationships: is a type of peroxisome organization [GO:0007031]; is a type of GO:0033365 Subtypes: GO:0016558, protein import into peroxisome membrane [GO:0045046], GO:0106101 Definition: A process in which a protein is transported to, or maintained at, a location in a peroxisome. Sources: GOC:ecd Also known as: protein localisation to peroxisome